{
  "gene": "UniProtKB:Q8NCE2",
  "term_id": "UNKNOWN:0002",
  "gene_name": "Myotubularin-related protein 14",
  "term_label": "Unknown biological process",
  "gene_symbol": "MTMR14"
}